L-asparagine catabolic process [GO:0006530] (biological process) Also known as: asparagine breakdown, asparagine catabolism, asparagine degradation Definition: The chemical reactions and pathways resulting in the breakdown of L-asparagine, 2-amino-3-carbamoylpropanoic acid. Relationships: is a type of L-asparagine metabolic process [GO:0070982]; is a type of L-amino acid catabolic process [GO:0170035]; is a type of proteinogenic amino acid catabolic process [GO:0170040] Sources: GOC:go_curators Subtypes: L-asparagine catabolic process via L-aspartate [GO:0033345], L-asparagine catabolic process via 2-oxosuccinamate [GO:0033346]